{
  "term_id": "GO:0035252",
  "gene": "UniProtKB:Q4G148",
  "gene_name": "Glucoside xylosyltransferase 1",
  "term_label": "UDP-xylosyltransferase activity",
  "gene_symbol": "GXYLT1"
}